2-dehydro-3-deoxy-L-pentonate aldolase activity [GO:0047438] (molecular function) Definition: Catalysis of the reaction: 2-dehydro-3-deoxy-L-pentonate = glycolaldehyde + pyruvate. Also known as: 3-deoxy-D-pentulosonic acid aldolase, 2-keto-3-deoxy-L-arabonate aldolase activity, 2-dehydro-3-deoxy-L-pentonate glycolaldehyde-lyase (pyruvate-forming), 2-dehydro-3-deoxy-L-pentonate glycolaldehyde-lyase activity, 2-keto-3-deoxy-D-xylonate aldolase activity, 2-keto-3-deoxy-L-pentonate aldolase activity Sources: EC:4.1.2.18, MetaCyc:4.1.2.18-RXN Relationships: is a type of aldehyde-lyase activity [GO:0016832]